(2Z,6Z)-farnesyl diphosphate synthase activity [GO:0102059] (molecular function) Definition: Catalysis of the reaction: 2 isopentenyl diphosphate + dimethylallyl diphosphate = (2Z,6Z)-farnesyl diphosphate + 2 diphosphate. Sources: RHEA:27810 Relationships: is a type of GO:0120531 Also known as: 2-cis,6-cis-farnesyl pyrophosphate synthase activity, Z,Z-FPP synthase activity, Z,Z-farnesyl pyrophosphate synthase activity, cis,cis-farnesyl diphosphate synthase activity, zFPS activity, neryl-diphosphate:isopentenyl-diphosphate cistransferase activity